response to parathyroid hormone [GO:0071107] (biological process) Relationships: is a type of response to hormone [GO:0009725] Definition: Any process that results in a change in state or activity of a cell or an organism (in terms of movement, secretion, enzyme production, gene expression, etc.) as a result of a parathyroid hormone stimulus. Also known as: response to parathyroid hormone stimulus Subtypes: cellular response to parathyroid hormone stimulus [GO:0071374] Sources: GOC:mah, GOC:yaf